negative regulation of asymmetric protein localization involved in cell fate determination [GO:1904786] (biological process) Definition: Any process that stops, prevents or reduces the frequency, rate or extent of asymmetric protein localization involved in cell fate determination. References: PMID:17476329 Sources: GOC:TermGenie, GO_REF:0000058 Also known as: down regulation of asymmetric protein localisation involved in cell fate determination, down regulation of asymmetric protein localization involved in cell fate commitment, down regulation of asymmetric protein localization involved in cell fate determination, down regulation of asymmetric protein localization resulting in cell fate commitment, down regulation of cell fate commitment, asymmetric protein localization, down-regulation of asymmetric protein localisation involved in cell fate determination, down-regulation of asymmetric protein localization involved in cell fate commitment, down-regulation of asymmetric protein localization involved in cell fate determination, down-regulation of asymmetric protein localization resulting in cell fate commitment, down-regulation of cell fate commitment, asymmetric protein localization, downregulation of asymmetric protein localisation involved in cell fate determination, downregulation of asymmetric protein localization involved in cell fate commitment, downregulation of asymmetric protein localization involved in cell fate determination, downregulation of asymmetric protein localization resulting in cell fate commitment, downregulation of cell fate commitment, asymmetric protein localization, negative regulation of asymmetric protein localisation involved in cell fate determination, negative regulation of asymmetric protein localization involved in cell fate commitment, negative regulation of asymmetric protein localization resulting in cell fate commitment, negative regulation of cell fate commitment, asymmetric protein localization, inhibition of asymmetric protein localisation involved in cell fate determination, inhibition of asymmetric protein localization involved in cell fate commitment, inhibition of asymmetric protein localization involved in cell fate determination, inhibition of asymmetric protein localization resulting in cell fate commitment, inhibition of cell fate commitment, asymmetric protein localization Note: wrm-1 in C. Elegans (Q10953) in PMID:17476329 (IMP) Relationships: is a type of negative regulation of protein localization [GO:1903828]; is a type of regulation of asymmetric protein localization involved in cell fate determination [GO:1904785]; negatively regulates GO:0045167